p-cresol catabolic process [GO:1901785] (biological process) References: PMID:10623531 Sources: GOC:TermGenie, GOC:yaf, UniPathway:UPA00708 Relationships: is a type of GO:0046199 Definition: The chemical reactions and pathways resulting in the breakdown of p-cresol. Also known as: p-cresol breakdown, p-cresol catabolism, p-cresol degradation